{
  "gene": "UniProtKB:Q9UNE7",
  "gene_name": "E3 ubiquitin-protein ligase CHIP",
  "gene_symbol": "STUB1",
  "term_label": "Z disc",
  "term_id": "GO:0030018"
}